death domain binding [GO:0070513] (molecular function) Subtypes: BH3 domain binding [GO:0051434] Definition: Binding to a death domain of a protein. The death domain (DD) is a homotypic protein interaction module composed of a bundle of six alpha-helices. DD bind each other forming oligomers. Some DD-containing proteins are involved in the regulation of apoptosis and inflammation through their activation of caspases and NF-kappaB. Note: For binding to the death effector domain, consider instead the term 'death effector domain binding ; GO:0035877'. Relationships: is a type of protein domain specific binding [GO:0019904] Sources: GOC:BHF, GOC:rl, InterPro:IPR000488, Pfam:PF00531